{
  "gene": "UniProtKB:O76090",
  "gene_symbol": "BEST1",
  "term_label": "plasma membrane",
  "gene_name": "Bestrophin-1",
  "term_id": "GO:0005886"
}